cell migration involved in metanephros development [GO:0035788] (biological process) Relationships: is a type of cell migration involved in kidney development [GO:0035787]; is part of GO:0001656 Definition: The orderly movement of a cell from one site to another that will contribute to the progression of the metanephric kidney over time, from its formation to the mature organ. Sources: GOC:bf, GOC:mtg_kidney_jan10, GOC:yaf Also known as: cell migration involved in metanephric kidney development Subtypes: metanephric mesenchymal cell migration [GO:0035789], epithelial cell migration involved in metanephric nephron tubule morphogenesis [GO:0072290]